{
  "term_label": "neuropeptide signaling pathway",
  "term_id": "GO:0007218",
  "gene": "UniProtKB:Q15722",
  "gene_symbol": "LTB4R",
  "gene_name": "Leukotriene B4 receptor 1"
}